{
  "term_label": "heterochromatin formation",
  "gene_name": "Transcription activator BRG1",
  "term_id": "GO:0031507",
  "gene_symbol": "SMARCA4",
  "gene": "UniProtKB:P51532"
}